negative regulation of collateral sprouting of injured axon [GO:0048695] (biological process) Sources: GOC:dgh, GOC:dph, GOC:jid, GOC:lm Also known as: down regulation of collateral sprouting of injured axon, down-regulation of collateral sprouting of injured axon, downregulation of collateral sprouting of injured axon, inhibition of collateral sprouting of injured axon Relationships: is a type of GO:0048671; is a type of GO:0048688; is a type of regulation of collateral sprouting of injured axon [GO:0048693]; RO_0002212 GO:0048674 Definition: Any process that stops, prevents, or reduces the frequency, rate or extent of collateral sprouting of an injured axon.